{
  "gene_symbol": "KATNAL1",
  "term_id": "GO:0005819",
  "term_label": "spindle",
  "gene_name": "Katanin p60 ATPase-containing subunit A-like 1",
  "gene": "UniProtKB:Q9BW62"
}